gamma-aminobutyric acid import [GO:0051939] (biological process) Sources: GOC:ai Also known as: 4-aminobutyrate import, GABA import, gamma-aminobutyrate import, gamma-aminobutyric acid uptake Definition: The directed movement of gamma-aminobutyric acid (GABA, 4-aminobutyrate) into a cell or organelle. Relationships: is a type of acidic amino acid transport [GO:0015800]; is a type of gamma-aminobutyric acid transport [GO:0015812]